arachidonate 15-lipoxygenase activity [GO:0050473] (molecular function) Also known as: 15-lipoxygenase activity, arachidonate omega(6) lipoxygenase activity, arachidonate omega6 lipoxygenase activity, arachidonate:oxygen 15-oxidoreductase activity, linoleic acid omega6-lipoxygenase activity, omega6 lipoxygenase activity Sources: EC:1.13.11.33 Definition: Catalysis of the reaction: arachidonate + O2 = (5Z,8Z,11Z,13E)-(15S)-15-hydroperoxyicosa-5,8,11,13-tetraenoate. Relationships: is a type of oxidoreductase activity, acting on single donors with incorporation of molecular oxygen, incorporation of two atoms of oxygen [GO:0016702]